{
  "gene_name": "SH3 and multiple ankyrin repeat domains protein 2",
  "term_id": "GO:0050808",
  "term_label": "synapse organization",
  "gene": "UniProtKB:Q9UPX8",
  "gene_symbol": "SHANK2"
}